{
  "term_label": "Unknown molecular function",
  "gene": "UniProtKB:Q5TEZ5",
  "gene_name": "Uncharacterized protein C6orf163",
  "term_id": "UNKNOWN:0001",
  "gene_symbol": "C6orf163"
}